{
  "gene_name": "Potassium voltage-gated channel subfamily D member 2",
  "term_id": "GO:0043197",
  "gene": "UniProtKB:Q9NZV8",
  "term_label": "dendritic spine",
  "gene_symbol": "KCND2"
}